follicle-stimulating hormone signaling pathway [GO:0042699] (biological process) Relationships: is a type of GO:0007186; is a type of ovulation cycle process [GO:0022602]; is part of ovarian follicle development [GO:0001541] Also known as: follicle stimulating hormone signaling pathway, follicle stimulating hormone signalling pathway, follicle-stimulating hormone signalling pathway Sources: GOC:dph Definition: A G protein-coupled receptor signaling pathway initiated by follicle-stimulating hormone binding to its receptor on the surface of a target cell, and ending with the regulation of a downstream cellular process.